CDP-diacylglycerol-glycerol-3-phosphate 3-phosphatidyltransferase activity [GO:0008444] (molecular function) Also known as: 3-phosphatidyl-1'-glycerol-3'-phosphate synthase activity, CDP-diacylglycerol:sn-glycerol-3-phosphate 3-phosphatidyltransferase activity, CDPdiacylglycerol-glycerol-3-phosphate 3-phosphatidyltransferase activity, CDPdiacylglycerol-sn-glycerol-3-phosphate 3-phosphatidyltransferase activity, CDPdiacylglycerol:glycerol-3-phosphate phosphatidyltransferase activity, CDPdiacylglycerol:sn-glycero-3-phosphate phosphatidyltransferase activity, PGP synthase activity, cytidine 5'-diphospho-1,2-diacyl-sn-glycerol (CDPdiglyceride):sn-glycerol-3-phosphate phosphatidyltransferase activity, glycerol 3-phosphate phosphatidyltransferase activity, glycerol phosphate phosphatidyltransferase activity, glycerophosphate phosphatidyltransferase activity, phosphatidylglycerol phosphate synthase activity, phosphatidylglycerol phosphate synthetase activity, phosphatidylglycerolphosphate synthase activity, phosphatidylglycerophosphate synthase activity, phosphatidylglycerophosphate synthetase activity, sn-glycerol-3-phosphate phosphatidyltransferase activity Relationships: is a type of CDP-alcohol phosphatidyltransferase activity [GO:0017169] Sources: EC:2.7.8.5, RHEA:12593 Definition: Catalysis of the reaction: sn-glycerol 3-phosphate + CDP-diacylglycerol = 3-(3-sn-phosphatidyl)-sn-glycerol 1-phosphate + CMP + H+.